manganese ion homeostasis [GO:0055071] (biological process) Definition: Any process involved in the maintenance of an internal steady state of manganese ions within an organism or cell. Sources: GOC:jid, GOC:mah Also known as: manganese homeostasis Relationships: is a type of monoatomic cation homeostasis [GO:0055080]; is a type of inorganic ion homeostasis [GO:0098771] Subtypes: intracellular manganese ion homeostasis [GO:0030026]